{
  "gene": "UniProtKB:Q6P4A8",
  "gene_symbol": "PLBD1",
  "gene_name": "Phospholipase B-like 1",
  "term_id": "GO:0005576",
  "term_label": "extracellular region"
}